{
  "term_label": "phosphatidylinositol-4,5-bisphosphate binding",
  "term_id": "GO:0005546",
  "gene": "UniProtKB:Q9Y6U3",
  "gene_symbol": "SCIN",
  "gene_name": "Scinderin"
}